{
  "gene": "UniProtKB:P49005",
  "term_label": "DNA strand elongation involved in DNA replication",
  "gene_symbol": "POLD2",
  "gene_name": "DNA polymerase delta subunit 2",
  "term_id": "GO:0006271"
}